{
  "term_label": "regulation of transcription by RNA polymerase II",
  "gene": "UniProtKB:Q99684",
  "term_id": "GO:0006357",
  "gene_name": "Zinc finger protein Gfi-1",
  "gene_symbol": "GFI1"
}